{
  "gene_symbol": "GGACT",
  "term_label": "Unknown molecular function",
  "gene": "UniProtKB:Q9BVM4",
  "gene_name": "Gamma-glutamylaminecyclotransferase",
  "term_id": "UNKNOWN:0001"
}